{
  "gene_symbol": "RHOT2",
  "gene_name": "Mitochondrial Rho GTPase 2",
  "gene": "UniProtKB:Q8IXI1",
  "term_label": "GTPase activity",
  "term_id": "GO:0003924"
}